{
  "gene_symbol": "ZNF562",
  "gene_name": "Zinc finger protein 562",
  "term_id": "GO:0006355",
  "gene": "UniProtKB:Q6V9R5",
  "term_label": "regulation of DNA-templated transcription"
}